{
  "gene": "UniProtKB:Q9NZ52",
  "gene_name": "ADP-ribosylation factor-binding protein GGA3",
  "term_label": "protein localization to cell surface",
  "term_id": "GO:0034394",
  "gene_symbol": "GGA3"
}